{
  "gene_name": "Vomeronasal type-1 receptor 1",
  "term_id": "GO:0005550",
  "term_label": "pheromone binding",
  "gene": "UniProtKB:Q9GZP7",
  "gene_symbol": "VN1R1"
}